{
  "term_id": "GO:1990904",
  "gene_symbol": "HNRNPF",
  "gene": "UniProtKB:P52597",
  "gene_name": "Heterogeneous nuclear ribonucleoprotein F",
  "term_label": "ribonucleoprotein complex"
}